deoxyuridine phosphorylase activity [GO:0047847] (MF) Definition: Catalysis of the reaction: 2'-deoxyuridine + phosphate = 2-deoxy-alpha-D-ribose 1-phosphate + uracil. Sources: RHEA:22824 Relationships: is a type of GO:0016154